{
  "term_label": "Unknown molecular function",
  "gene_symbol": "LRRD1",
  "term_id": "UNKNOWN:0001",
  "gene": "UniProtKB:A4D1F6",
  "gene_name": "Leucine-rich repeat and death domain-containing protein 1"
}